{
  "gene_symbol": "RALA",
  "term_label": "Ras protein signal transduction",
  "gene": "UniProtKB:P11233",
  "term_id": "GO:0007265",
  "gene_name": "Ras-related protein Ral-A"
}